{
  "gene": "UniProtKB:Q5T5B0",
  "gene_symbol": "LCE3E",
  "term_label": "Unknown cellular component",
  "gene_name": "Late cornified envelope protein 3E",
  "term_id": "UNKNOWN:0003"
}